{
  "gene_symbol": "DNTT",
  "term_label": "nucleus",
  "term_id": "GO:0005634",
  "gene_name": "DNA nucleotidylexotransferase",
  "gene": "UniProtKB:P04053"
}